{
  "term_label": "inflammatory response",
  "term_id": "GO:0006954",
  "gene_symbol": "AFAP1L2",
  "gene_name": "Actin filament-associated protein 1-like 2",
  "gene": "UniProtKB:Q8N4X5"
}